{
  "term_label": "Unknown molecular function",
  "term_id": "UNKNOWN:0001",
  "gene": "UniProtKB:Q5SQH8",
  "gene_name": "Uncharacterized protein C6orf136",
  "gene_symbol": "C6orf136"
}